glycine betaine transport [GO:0031460] (biological process) Definition: The directed movement of glycine betaine, N-trimethylglycine, into, out of or within a cell, or between cells, by means of some agent such as a transporter or pore. Also known as: N-trimethylglycine transport Sources: GOC:mah Relationships: is a type of GO:0015695; is a type of GO:0015838